{
  "gene_symbol": "ETV5",
  "gene_name": "ETS translocation variant 5",
  "term_label": "cell differentiation",
  "gene": "UniProtKB:P41161",
  "term_id": "GO:0030154"
}